negative regulation of cerebral blood circulation [GO:0120278] (biological process) Relationships: is a type of regulation of cerebral blood circulation [GO:0120276]; is a type of negative regulation of blood circulation [GO:1903523]; negatively regulates cerebral blood circulation [GO:0120275] References: PMID:25397684 Sources: GOC:krc Also known as: down regulation of cerebral blood circulation, down-regulation of cerebral blood circulation, downregulation of cerebral blood circulation, negative regulation of cerebrum blood circulation, negative regulation of telencephalon blood circulation, inhibition of cerebral blood circulation Definition: Any process that stops, prevents or reduces the frequency, rate or extent of cerebral blood circulation.